T cell homeostatic proliferation [GO:0001777] (biological process) Regulation: positively regulated by GO:0042103; regulated by regulation of T cell homeostatic proliferation [GO:0046013]; negatively regulated by GO:0046014 Definition: The non-specific expansion of T cell populations within a whole or part of an organism to reach to a total number of T cells which will then remain stable over time in the absence of an external stimulus. Also known as: T lymphocyte homeostatic proliferation, T-cell homeostatic proliferation, T-lymphocyte homeostatic proliferation, resting T cell proliferation, resting T-cell proliferation Relationships: is a type of T cell proliferation [GO:0042098]; is part of T cell homeostasis [GO:0043029] Sources: GOC:mgi_curators, ISBN:0781735149